{
  "gene_symbol": "MFSD9",
  "term_id": "UNKNOWN:0001",
  "gene_name": "Major facilitator superfamily domain-containing protein 9",
  "term_label": "Unknown molecular function",
  "gene": "UniProtKB:Q8NBP5"
}